{
  "term_id": "GO:0005044",
  "gene_symbol": "SCARF1",
  "gene_name": "Scavenger receptor class F member 1",
  "term_label": "scavenger receptor activity",
  "gene": "UniProtKB:Q14162"
}